D-xylose metabolic process [GO:0042732] (biological process) Relationships: is a type of pentose metabolic process [GO:0019321] Sources: ISBN:0198506732 Also known as: D-xylose metabolism Subtypes: D-xylose biosynthetic process [GO:0042842], D-xylose catabolic process [GO:0042843] Definition: The chemical reactions and pathways involving D-xylose, a naturally occurring plant polysaccharide.